{
  "gene_name": "Teneurin-1",
  "term_id": "GO:0046982",
  "term_label": "protein heterodimerization activity",
  "gene": "UniProtKB:Q9UKZ4",
  "gene_symbol": "TENM1"
}